regulation of leaf morphogenesis [GO:1901371] (biological process) Definition: Any process that modulates the frequency, rate or extent of leaf morphogenesis. Subtypes: regulation of leaflet formation [GO:0090016] Sources: GOC:TermGenie Relationships: is a type of regulation of shoot system morphogenesis [GO:1900618]; is a type of regulation of plant organ morphogenesis [GO:1905421]; regulates leaf morphogenesis [GO:0009965]